catecholamine biosynthetic process [GO:0042423] (BP) Also known as: catecholamine anabolism, catecholamine biosynthesis, catecholamine formation, catecholamine synthesis Relationships: is a type of catecholamine metabolic process [GO:0006584]; is a type of catechol-containing compound biosynthetic process [GO:0009713]; is a type of biogenic amine biosynthetic process [GO:0042401] Subtypes: GO:0042416, epinephrine biosynthetic process [GO:0042418], norepinephrine biosynthetic process [GO:0042421] Definition: The chemical reactions and pathways resulting in the formation of any of a group of physiologically important biogenic amines that possess a catechol (3,4-dihydroxyphenyl) nucleus and are derivatives of 3,4-dihydroxyphenylethylamine. Sources: GOC:jl, ISBN:0198506732